{
  "term_id": "GO:0042148",
  "gene_symbol": "DMC1",
  "term_label": "DNA strand invasion",
  "gene_name": "Meiotic recombination protein DMC1_LIM15 homolog",
  "gene": "UniProtKB:Q14565"
}